oligodendrocyte cell fate specification [GO:0021778] (biological process) Subtypes: spinal cord oligodendrocyte cell fate specification [GO:0021530] Definition: The process in which a cell becomes capable of differentiating autonomously into an oligodendrocyte in an environment that is neutral with respect to the developmental pathway. Upon specification, the cell fate can be reversed. Sources: GOC:cls, GOC:dgh, GOC:dph, GOC:jid, GO_REF:0000021 Relationships: is a type of glial cell fate specification [GO:0021780]; is part of GO:0021779